swim bladder maturation [GO:0048796] (biological process) Also known as: gas bladder maturation Sources: GOC:devbiol Definition: A developmental process, independent of morphogenetic (shape) change, that is required for a swim bladder to attain its fully functional state. The swim bladder is used by some fishes to maintain buoyancy and may function in addition as a sound producing organ, a sound receptor, and a respiratory organ. Relationships: is_a animal organ maturation [GO:0048799]; is part of swim bladder development [GO:0048794]